{
  "gene_name": "Protein mono-ADP-ribosyltransferase PARP9",
  "term_id": "GO:0005737",
  "term_label": "cytoplasm",
  "gene": "UniProtKB:Q8IXQ6",
  "gene_symbol": "PARP9"
}